{
  "term_id": "UNKNOWN:0003",
  "gene_symbol": "COPS9",
  "gene": "UniProtKB:Q8WXC6",
  "gene_name": "COP9 signalosome complex subunit 9",
  "term_label": "Unknown cellular component"
}